{
  "gene_symbol": "CMTM3",
  "term_label": "Unknown molecular function",
  "gene": "UniProtKB:Q96MX0",
  "gene_name": "CKLF-like MARVEL transmembrane domain-containing protein 3",
  "term_id": "UNKNOWN:0001"
}